cellular response to glucocorticoid stimulus [GO:0071385] (biological process) Relationships: is a type of response to glucocorticoid [GO:0051384]; is a type of cellular response to corticosteroid stimulus [GO:0071384] Subtypes: cellular response to corticosterone stimulus [GO:0071386], GO:0071387, cellular response to cortisone stimulus [GO:0071388], cellular response to dexamethasone stimulus [GO:0071549] Sources: GOC:mah Definition: Any process that results in a change in state or activity of a cell (in terms of movement, secretion, enzyme production, gene expression, etc.) as a result of a glucocorticoid stimulus. Glucocorticoids are hormonal C21 corticosteroids synthesized from cholesterol with the ability to bind with the cortisol receptor and trigger similar effects. Glucocorticoids act primarily on carbohydrate and protein metabolism, and have anti-inflammatory effects.